negative regulation of lipopolysaccharide-mediated signaling pathway [GO:0031665] (biological process) Relationships: is a type of negative regulation of response to biotic stimulus [GO:0002832]; is a type of GO:0009968; is_a GO:0031664; is a type of negative regulation of response to external stimulus [GO:0032102]; negatively regulates lipopolysaccharide-mediated signaling pathway [GO:0031663] Sources: GOC:mah Also known as: down regulation of lipopolysaccharide-mediated signaling pathway, down-regulation of lipopolysaccharide-mediated signaling pathway, downregulation of lipopolysaccharide-mediated signaling pathway, negative regulation of LPS-mediated signaling pathway, negative regulation of lipopolysaccharide-mediated signalling pathway, inhibition of lipopolysaccharide-mediated signaling pathway Definition: Any process that stops, prevents, or reduces the frequency, rate or extent of signaling in response to detection of lipopolysaccharide. Subtypes: tolerance induction to lipopolysaccharide [GO:0072573]